{
  "gene_name": "Hypoxia up-regulated protein 1",
  "term_id": "GO:0034663",
  "gene": "UniProtKB:Q9Y4L1",
  "gene_symbol": "HYOU1",
  "term_label": "endoplasmic reticulum chaperone complex"
}